{
  "gene_name": "Putative protein FAM90A5P",
  "gene_symbol": "FAM90A5P",
  "term_id": "UNKNOWN:0002",
  "term_label": "Unknown biological process",
  "gene": "UniProtKB:A8MXJ8"
}